{
  "term_id": "UNKNOWN:0001",
  "gene_name": "NHS-like protein 2",
  "gene": "UniProtKB:Q5HYW2",
  "gene_symbol": "NHSL2",
  "term_label": "Unknown molecular function"
}